{
  "term_id": "GO:0004725",
  "term_label": "protein tyrosine phosphatase activity",
  "gene_symbol": "DUSP21",
  "gene": "UniProtKB:Q9H596",
  "gene_name": "Dual specificity protein phosphatase 21"
}